{
  "term_id": "UNKNOWN:0002",
  "term_label": "Unknown biological process",
  "gene_symbol": "UNC50",
  "gene_name": "Protein unc-50 homolog",
  "gene": "UniProtKB:Q53HI1"
}